all-trans-retinyl-ester hydrolase, 11-cis retinol forming activity [GO:0052885] (molecular function) Relationships: is a type of carboxylic ester hydrolase activity [GO:0052689]; is part of retinol metabolic process [GO:0042572] Definition: Catalysis of the reaction: H2O + all-trans-retinyl ester = 11-cis-retinol + fatty acid. Regulation: negatively regulated by GO:0062003 Also known as: all-trans-retinol isomerase:hydrolase activity, retinoid isomerohydrolase activity, retinol isomerase activity, all-trans-retinyl ester acylhydrolase, 11-cis retinol forming activity, all-trans-retinylester 11-cis isomerohydrolase activity Sources: RHEA:31771